{
  "gene_name": "Homeobox protein Hox-C9",
  "gene_symbol": "HOXC9",
  "term_label": "DNA-binding transcription factor activity",
  "gene": "UniProtKB:P31274",
  "term_id": "GO:0003700"
}